{
  "gene_symbol": "ATP6AP1",
  "term_label": "proton-transporting V-type ATPase complex",
  "gene_name": "V-type proton ATPase subunit S1",
  "term_id": "GO:0033176",
  "gene": "UniProtKB:Q15904"
}